{
  "gene_symbol": "OR9G9",
  "term_id": "UNKNOWN:0001",
  "gene_name": "Olfactory receptor 9G9",
  "gene": "UniProtKB:P0C7N8",
  "term_label": "Unknown molecular function"
}